epoxide metabolic process [GO:0097176] (biological process) Definition: The chemical reactions and pathways involving epoxides, compounds in which an oxygen atom is directly attached to two adjacent or non-adjacent carbon atoms of a carbon chain or ring system; thus cyclic ethers. References: PMID:15822179 Sources: GOC:rs Relationships: is a type of metabolic process [GO:0008152] Also known as: epoxide metabolism Subtypes: tetrahydrofuran catabolic process [GO:0018968], GO:0019639, vomitoxin biosynthetic process [GO:0106110], scopolamine biosynthetic process [GO:1900991], leukotriene A4 metabolic process [GO:1901751], GO:1901779, pentalenolactone biosynthetic process [GO:1901780], GO:1901802, GO:1901803, all-trans-neoxanthin catabolic process [GO:1901832], neoxanthin biosynthetic process [GO:1901833], fumagillin catabolic process [GO:1902085], fumagillin biosynthetic process [GO:1902086]